{
  "gene_name": "Centrin-2",
  "term_id": "GO:0000226",
  "gene": "UniProtKB:P41208",
  "gene_symbol": "CETN2",
  "term_label": "microtubule cytoskeleton organization"
}